catechol 1,2-dioxygenase activity [GO:0018576] (molecular function) Also known as: 1,2-pyrocatechase activity, CD I, CD II, catechase activity, catechol 1,2-oxygenase activity, catechol-oxygen 1,2-oxidoreductase activity, catechol:oxygen 1,2-oxidoreductase activity, pyrocatechase activity, pyrocatechol 1,2-dioxygenase activity Sources: RHEA:23852 Relationships: is a type of oxidoreductase activity, acting on single donors with incorporation of molecular oxygen, incorporation of two atoms of oxygen [GO:0016702] Definition: Catalysis of the reaction: catechol + O2 = cis,cis-muconate.